regulation of type 2 mitophagy [GO:1905089] (biological process) References: PMID:26942284 Definition: Any process that modulates the frequency, rate or extent of type 2 mitophagy. Relationships: is a type of regulation of mitophagy [GO:1901524]; regulates type 2 mitophagy [GO:0061734] Subtypes: GO:1905090, positive regulation of type 2 mitophagy [GO:1905091] Also known as: regulation of PRKN-mediated stimulation of mitophagy in response to mitochondrial depolarization, regulation of Park2-mediated stimulation of mitophagy in response to mitochondrial depolarization, regulation of parkin-mediated stimulation of mitophagy in response to mitochondrial depolarization